{
  "gene": "UniProtKB:A6NMB9",
  "term_id": "GO:0051013",
  "gene_name": "Fidgetin-like protein 2",
  "term_label": "microtubule severing",
  "gene_symbol": "FIGNL2"
}